{
  "term_id": "GO:0050852",
  "gene_name": "Tyrosine-protein kinase Tec",
  "gene": "UniProtKB:P42680",
  "gene_symbol": "TEC",
  "term_label": "T cell receptor signaling pathway"
}